positive regulation of translational initiation by iron [GO:0045994] (biological process) Relationships: is_a regulation of translational initiation by iron [GO:0006447]; is a type of positive regulation of translational initiation [GO:0045948] Also known as: up regulation of translational initiation by iron, up-regulation of translational initiation by iron, upregulation of translational initiation by iron, activation of translational initiation by iron, stimulation of translational initiation by iron Sources: GOC:go_curators Definition: Any process involving iron that activates or increases the rate of translational initiation.